{
  "term_id": "GO:0005096",
  "term_label": "GTPase activator activity",
  "gene_symbol": "SIPA1",
  "gene_name": "Signal-induced proliferation-associated protein 1",
  "gene": "UniProtKB:Q96FS4"
}